{
  "gene_symbol": "MC4R",
  "term_label": "melanocyte-stimulating hormone receptor activity",
  "gene_name": "Melanocortin receptor 4",
  "gene": "UniProtKB:P32245",
  "term_id": "GO:0004980"
}